mitochondrial electron transport, NADH to ubiquinone [GO:0006120] (biological process) Definition: The transfer of electrons from NADH to ubiquinone that occurs during oxidative phosphorylation. Sources: ISBN:0716731363 Regulation: regulated by GO:1902956; negatively regulated by negative regulation of mitochondrial electron transport, NADH to ubiquinone [GO:1902957]; positively regulated by positive regulation of mitochondrial electron transport, NADH to ubiquinone [GO:1902958] Also known as: oxidative phosphorylation, NADH to ubiquinone, complex I (NADH to ubiquinone) Relationships: is a type of aerobic electron transport chain [GO:0019646]; is part of mitochondrial ATP synthesis coupled electron transport [GO:0042775]